{
  "gene_symbol": "RPA3",
  "term_label": "base-excision repair",
  "gene_name": "Replication protein A 14 kDa subunit",
  "term_id": "GO:0006284",
  "gene": "UniProtKB:P35244"
}